{
  "term_label": "Unknown biological process",
  "term_id": "UNKNOWN:0002",
  "gene_name": "T cell receptor gamma joining 2 (Fragment)",
  "gene_symbol": "TRGJ2",
  "gene": "UniProtKB:A0A5H1ZRR4"
}